cyclohexanone dehydrogenase activity [GO:0047797] (molecular function) Sources: EC:1.3.99.14, RHEA:21780 Definition: Catalysis of the reaction: A + cyclohexanone = AH(2) + cyclohex-2-enone. Relationships: is a type of oxidoreductase activity, acting on the CH-CH group of donors [GO:0016627] Also known as: cyclohexanone:(acceptor) 2-oxidoreductase activity, cyclohexanone:acceptor 2-oxidoreductase activity